{
  "gene": "UniProtKB:Q8N9F0",
  "term_id": "GO:0031966",
  "gene_name": "N-acetylaspartate synthetase",
  "term_label": "mitochondrial membrane",
  "gene_symbol": "NAT8L"
}